{
  "gene_symbol": "TBC1D3",
  "gene_name": "TBC1 domain family member 3",
  "gene": "UniProtKB:Q8IZP1",
  "term_id": "GO:0005096",
  "term_label": "GTPase activator activity"
}